{
  "term_id": "UNKNOWN:0001",
  "term_label": "Unknown molecular function",
  "gene_name": "Pleckstrin homology domain-containing family H member 1",
  "gene_symbol": "PLEKHH1",
  "gene": "UniProtKB:Q9ULM0"
}